{
  "gene_name": "Interferon alpha-2",
  "gene": "UniProtKB:P01563",
  "term_id": "GO:0005132",
  "term_label": "type I interferon receptor binding",
  "gene_symbol": "IFNA2"
}